phosphotransferase activity, paired acceptors [GO:0016781] (molecular function) Subtypes: GO:0004756, GO:0008986, GO:0050242, GO:0050521, GO:0051752 Relationships: is a type of transferase activity, transferring phosphorus-containing groups [GO:0016772] Definition: Catalysis of the transfer of two phosphate groups from a donor, such as ATP, to two different acceptors. Sources: EC:2.7.9.-